positive regulation of taurine biosynthetic process [GO:0062090] (biological process) References: PMID:18648510, PMID:24911144 Sources: GOC:BHF Definition: Any process that activates or increases the frequency, rate or extent of taurine biosynthesis. Relationships: is a type of positive regulation of biosynthetic process [GO:0009891]; is a type of positive regulation of small molecule metabolic process [GO:0062013]; is a type of regulation of taurine biosynthetic process [GO:0062089]; positively regulates taurine biosynthetic process [GO:0042412]